{
  "term_label": "Unknown biological process",
  "gene_name": "Olfactory receptor 52A5",
  "gene": "UniProtKB:Q9H2C5",
  "gene_symbol": "OR52A5",
  "term_id": "UNKNOWN:0002"
}